{
  "term_id": "UNKNOWN:0002",
  "gene_symbol": "EVI5L",
  "gene_name": "EVI5-like protein",
  "term_label": "Unknown biological process",
  "gene": "UniProtKB:Q96CN4"
}